{
  "gene_symbol": "DKK2",
  "term_label": "negative regulation of canonical Wnt signaling pathway",
  "term_id": "GO:0090090",
  "gene": "UniProtKB:Q9UBU2",
  "gene_name": "Dickkopf-related protein 2"
}